{
  "gene_name": "Coiled-coil domain-containing protein 144A",
  "gene": "UniProtKB:A2RUR9",
  "gene_symbol": "CCDC144A",
  "term_label": "Unknown cellular component",
  "term_id": "UNKNOWN:0003"
}